{
  "gene_name": "Ovochymase-1",
  "term_label": "Unknown biological process",
  "gene": "UniProtKB:Q7RTY7",
  "term_id": "UNKNOWN:0002",
  "gene_symbol": "OVCH1"
}